L-kynurenine transmembrane transporter activity [GO:0140926] (molecular function) Definition: Enables the transfer of L-kynurenine from one side of a membrane to the other. Relationships: is a type of L-amino acid transmembrane transporter activity [GO:0015179]; is part of GO:0140924 References: PMID:35245456